phosphatidylinositol phosphate 5-phosphatase activity [GO:0034595] (molecular function) Also known as: phosphoinositide 5-phosphatase activity, polyphosphoinositol lipid 5-phosphatase activity Definition: Catalysis of the removal of the 5-phosphate group of a phosphatidylinositol phosphate. Relationships: is a type of phosphatidylinositol phosphate phosphatase activity [GO:0052866] Subtypes: phosphatidylinositol-4,5-bisphosphate 5-phosphatase activity [GO:0004439], phosphatidylinositol-3,4,5-trisphosphate 5-phosphatase activity [GO:0034485], phosphatidylinositol-3,5-bisphosphate 5-phosphatase activity [GO:0043813], phosphatidylinositol-1,4,5-trisphosphate 5-phosphatase activity [GO:0052867], GO:0102091 Sources: GOC:elh